corticospinal neuron axon guidance through the cerebral peduncle [GO:0021969] (BP) References: PMID:9878731 Sources: GOC:cls, GOC:dgh, GOC:dph, GOC:jid, GO_REF:0000021 Relationships: is a type of axon guidance [GO:0007411]; is part of corticospinal neuron axon guidance [GO:0021966] Definition: The process in which the migration of an axon growth cone of a pyramidal cell that is part of the corticospinal tract is directed after exiting the internal capsule through the cerebral peduncle in response to a combination of attractive and repulsive cues. Also known as: corticospinal neuron axon pathfinding through the cerebral peduncle